Ala-tRNA(Pro) deacylase activity [GO:0043906] (molecular function) References: PMID:14663147 Sources: GOC:jl Also known as: Ala-tRNAPro hydrolase activity Relationships: is_a GO:0002161 Definition: Catalysis of the hydrolysis of misacylated Ala-tRNA(Pro).